{
  "term_label": "SCF ubiquitin ligase complex",
  "term_id": "GO:0019005",
  "gene_symbol": "FBXO32",
  "gene_name": "F-box only protein 32",
  "gene": "UniProtKB:Q969P5"
}